{
  "gene_name": "Immunity-related GTPase family Q protein",
  "gene_symbol": "IRGQ",
  "term_id": "UNKNOWN:0002",
  "term_label": "Unknown biological process",
  "gene": "UniProtKB:Q8WZA9"
}